dynein axonemal particle [GO:0120293] (cellular component) Definition: An aggregation of axonemal dyneins, their specific assembly factors, and broadly-acting chaperones that is located in the cytoplasm. References: PMID:30561330, PMID:32898505, PMID:33263282 Sources: GOC:krc Also known as: DynAP Relationships: is a type of intracellular membraneless organelle [GO:0043232]; is part of cytoplasm [GO:0005737]